{
  "gene_name": "Alpha-parvin",
  "gene_symbol": "PARVA",
  "term_label": "establishment or maintenance of cell polarity regulating cell shape",
  "gene": "UniProtKB:Q9NVD7",
  "term_id": "GO:0071963"
}